L-threonine catabolic process to propionate [GO:0070689] (biological process) Relationships: is a type of L-threonine catabolic process [GO:0006567]; is a type of GO:0019541 Also known as: threonine catabolic process to propionate, L-threonine breakdown to propionate, L-threonine catabolism to propionate, L-threonine degradation to propionate Definition: The chemical reactions and pathways resulting in the breakdown of L-threonine (the L-enantiomer of 2-amino-3-hydroxybutyric acid) to form the compound propionate. Sources: GOC:bf, GOC:mah, MetaCyc:PWY-5437